{
  "term_label": "signal transduction",
  "term_id": "GO:0007165",
  "gene": "UniProtKB:Q8NEG4",
  "gene_symbol": "FAM83F",
  "gene_name": "Protein FAM83F"
}